{
  "gene": "UniProtKB:A8MTI9",
  "gene_symbol": "PRSS47P",
  "term_label": "proteolysis",
  "term_id": "GO:0006508",
  "gene_name": "Putative serine protease 47"
}